{
  "term_label": "Cul2-RING ubiquitin ligase complex",
  "gene_name": "Zinc finger SWIM domain-containing protein 4",
  "gene": "UniProtKB:Q9H7M6",
  "term_id": "GO:0031462",
  "gene_symbol": "ZSWIM4"
}